citronellyl-CoA ligase activity [GO:0034823] (molecular function) Definition: Catalysis of the reaction: citronellate + CoASH + ATP = citronellyl-CoA + AMP + PPi. Sources: UM-BBD_reactionID:r1157 Relationships: is a type of CoA-ligase activity [GO:0016405]; is a type of GO:0016878